{
  "gene_symbol": "KDM6B",
  "term_id": "GO:0000978",
  "term_label": "RNA polymerase II cis-regulatory region sequence-specific DNA binding",
  "gene": "UniProtKB:O15054",
  "gene_name": "Lysine-specific demethylase 6B"
}